{
  "gene": "UniProtKB:Q30KQ1",
  "gene_name": "Beta-defensin 133",
  "term_id": "GO:0060326",
  "gene_symbol": "DEFB133",
  "term_label": "cell chemotaxis"
}